glutamate synthase complex [GO:0031026] (cellular component) Relationships: is a type of GO:0140535; is a type of oxidoreductase complex [GO:1990204] Subtypes: glutamate synthase complex (NADPH) [GO:0009342], glutamate synthase complex (NADH) [GO:0031027] Definition: A complex that possesses glutamate synthase activity. Sources: GOC:mah